{
  "gene_symbol": "MORC3",
  "term_id": "GO:0140374",
  "gene_name": "MORC family CW-type zinc finger protein 3",
  "gene": "UniProtKB:Q14149",
  "term_label": "antiviral innate immune response"
}